{
  "gene_name": "Ubiquitin carboxyl-terminal hydrolase 17-like protein 6",
  "term_label": "regulation of protein stability",
  "gene_symbol": "USP17L6P",
  "gene": "UniProtKB:Q6QN14",
  "term_id": "GO:0031647"
}